ventriculo bulbo valve morphogenesis [GO:0003187] (BP) Relationships: is a type of GO:0003179; is part of ventriculo bulbo valve development [GO:0003173] Definition: The process in which the structure of the ventriculo bulbo valve is generated and organized. Sources: GOC:mtg_heart